{
  "gene_symbol": "SSX3",
  "term_id": "GO:0005634",
  "term_label": "nucleus",
  "gene_name": "Protein SSX3",
  "gene": "UniProtKB:Q99909"
}